retinoic acid 4-hydroxylase activity [GO:0008401] (molecular function) Subtypes: all-trans retinoic acid 4-hydrolase activity [GO:0062182] References: PMID:19519282, PMID:9250660 Definition: Catalysis of the conversion of retinoic acid to 4-hydroxy-retinoic acid. Also known as: cytochrome P450 CYP261 Relationships: is a type of GO:0004497; is a type of oxidoreductase activity, acting on paired donors, with incorporation or reduction of molecular oxygen [GO:0016705]